anterior mRNA localization involved in anterior/posterior axis specification [GO:0060813] (biological process) Also known as: anterior mRNA localisation involved in anterior/posterior axis specification Relationships: is a type of intracellular mRNA localization involved in anterior/posterior axis specification [GO:0060811] Definition: Any process in which a mRNA is transported to, and maintained in the anterior portion of the oocyte and/or syncytial embryo contributing to the specification of the anterior/posterior axis. Sources: GOC:dph, GOC:sdb_2009, GOC:tb